{
  "gene": "UniProtKB:Q9NQ87",
  "term_id": "GO:0005634",
  "gene_symbol": "HEYL",
  "gene_name": "Hairy_enhancer-of-split related with YRPW motif-like protein",
  "term_label": "nucleus"
}